{
  "term_label": "microtubule binding",
  "gene_name": "Kinesin-like protein KIFC1",
  "gene_symbol": "KIFC1",
  "term_id": "GO:0008017",
  "gene": "UniProtKB:Q9BW19"
}